{
  "gene_name": "Endothelin-2",
  "gene_symbol": "EDN2",
  "gene": "UniProtKB:P20800",
  "term_label": "extracellular space",
  "term_id": "GO:0005615"
}